{
  "gene": "UniProtKB:Q15822",
  "term_label": "neuron projection",
  "term_id": "GO:0043005",
  "gene_name": "Neuronal acetylcholine receptor subunit alpha-2",
  "gene_symbol": "CHRNA2"
}